{
  "gene": "UniProtKB:Q5BJE1",
  "gene_symbol": "CCDC178",
  "gene_name": "Coiled-coil domain-containing protein 178",
  "term_id": "UNKNOWN:0001",
  "term_label": "Unknown molecular function"
}